beta-adrenergic receptor kinase activity [GO:0047696] (molecular function) Sources: RHEA:19429 Relationships: is a type of protein kinase activity [GO:0004672] Definition: Catalysis of the reaction: [beta-adrenergic receptor] + ATP = [beta-adrenergic receptor]-phosphate + ADP + H+. Also known as: ATP:beta-adrenergic-receptor phosphotransferase activity, adrenergic receptor kinase activity, beta-adrenoceptor kinase 1 activity, beta-adrenoceptor kinase 2 activity, ADRBK1, BARK1, GRK2, GRK3, STK15, [b-adrenergic-receptor] kinase activity, beta-AR kinase activity, beta-ARK, beta-ARK 1, beta-ARK 2, beta-adrenergic receptor-specific kinase activity, beta-adrenergic-receptor kinase (phosphorylating) activity, beta-adrenergic-receptor kinase activity, beta-adrenoceptor kinase activity, beta-receptor kinase activity, beta2ARK, betaARK1